negative regulation of chromatin looping [GO:0160164] (biological process) Relationships: is a type of negative regulation of chromatin organization [GO:1905268]; negatively regulates chromatin looping [GO:0140588] Definition: Any process that stops, prevents or reduces the frequency, rate or extent of chromatin looping. References: PMID:34856126